phosphoric triester hydrolase activity [GO:0016795] (molecular function) Subtypes: aryldialkylphosphatase activity [GO:0004063] Definition: Catalysis of the hydrolysis of a phosphoric triester. Relationships: is a type of phosphoric ester hydrolase activity [GO:0042578] Sources: EC:3.1.8.-, GOC:curators